{
  "gene_symbol": "MAP1LC3B2",
  "term_label": "autophagosome assembly",
  "term_id": "GO:0000045",
  "gene": "UniProtKB:A6NCE7",
  "gene_name": "Microtubule-associated proteins 1A_1B light chain 3 beta 2"
}